{
  "gene_name": "Ubiquitin carboxyl-terminal hydrolase 21",
  "term_id": "GO:0005737",
  "gene_symbol": "USP21",
  "gene": "UniProtKB:Q9UK80",
  "term_label": "cytoplasm"
}